{
  "gene_name": "Butyrophilin-like protein 8",
  "term_label": "signaling receptor binding",
  "gene_symbol": "BTNL8",
  "term_id": "GO:0005102",
  "gene": "UniProtKB:Q6UX41"
}